transport of virus [GO:0046794] (BP) Relationships: is_a viral process [GO:0016032] Subtypes: transport of virus in multicellular host [GO:0046739], intracellular transport of virus [GO:0075733] Also known as: viral transport, virion transport Sources: GOC:ai Definition: The directed movement of a virus, or part of a virus, into, out of, or within a host cell.